{
  "gene_name": "Protein MTSS 1",
  "term_id": "GO:0032233",
  "gene_symbol": "MTSS1",
  "term_label": "positive regulation of actin filament bundle assembly",
  "gene": "UniProtKB:O43312"
}